{
  "gene_name": "5-hydroxytryptamine receptor 6",
  "gene_symbol": "HTR6",
  "term_label": "plasma membrane",
  "gene": "UniProtKB:P50406",
  "term_id": "GO:0005886"
}